{
  "gene_name": "Lysine-specific demethylase 2B",
  "term_label": "chromatin remodeling",
  "gene_symbol": "KDM2B",
  "term_id": "GO:0006338",
  "gene": "UniProtKB:Q8NHM5"
}